{
  "gene_name": "Serine_threonine-protein kinase tousled-like 1",
  "term_label": "chromosome segregation",
  "gene": "UniProtKB:Q9UKI8",
  "term_id": "GO:0007059",
  "gene_symbol": "TLK1"
}